{
  "gene_name": "Transmembrane protein 117",
  "gene_symbol": "TMEM117",
  "term_id": "UNKNOWN:0001",
  "gene": "UniProtKB:Q9H0C3",
  "term_label": "Unknown molecular function"
}